{
  "gene_symbol": "AOX1",
  "term_label": "Unknown cellular component",
  "gene": "UniProtKB:Q06278",
  "term_id": "UNKNOWN:0003",
  "gene_name": "Aldehyde oxidase"
}